{
  "term_id": "GO:0007015",
  "gene": "UniProtKB:P08134",
  "gene_symbol": "RHOC",
  "term_label": "actin filament organization",
  "gene_name": "Rho-related GTP-binding protein RhoC"
}